ovarian nurse cell to oocyte transport [GO:0007300] (biological process) Also known as: nurse cell to oocyte transport Definition: Transfer of constituents synthesized in the ovarian nurse cells to the oocyte, through the ring canals, as the egg chamber is growing. An example of this is found in Drosophila melanogaster. Relationships: is a type of GO:0006810; is part of oogenesis [GO:0048477] Sources: GOC:mtg_sensu, ISBN:0879694238